pilus tip [GO:0009419] (cellular component) Relationships: is a type of cellular anatomical structure [GO:0110165]; is part of pilus [GO:0009289] Sources: GOC:jl Definition: The pointed extremity furthest from the cell of a pilus. Also known as: fimbrial tip